SUMO conjugating enzyme activity [GO:0061656] (molecular function) Definition: Isoenergetic transfer of SUMO from one protein to another via the reaction X-SUMO + Y = Y-SUMO + X, where both the X-SUMO and Y-SUMO linkages are thioester bonds between the C-terminal amino acid of SUMO and a sulfhydryl side group of a cysteine residue. Sources: GOC:dph Also known as: E2 Relationships: is a type of SUMO transferase activity [GO:0019789]; is a type of ubiquitin-like protein conjugating enzyme activity [GO:0061650]